{
  "term_label": "myosin light chain kinase activity",
  "gene_symbol": "MYLK2",
  "gene_name": "Myosin light chain kinase 2, skeletal_cardiac muscle",
  "term_id": "GO:0004687",
  "gene": "UniProtKB:Q9H1R3"
}